linamarin synthase activity [GO:0050057] (molecular function) Sources: EC:2.4.1.63, MetaCyc:LINAMARIN-SYNTHASE-RXN Also known as: UDP glucose ketone cyanohydrin glucosyltransferase activity, UDP-glucose:2-hydroxy-2-methylpropanenitrile beta-D-glucosyltransferase activity, UDPglucose:2-hydroxy-2-methylpropanenitrile beta-D-glucosyltransferase activity, UDPglucose:ketone cyanohydrin beta-glucosyltransferase activity, uridine diphosphate-glucose-ketone cyanohydrin beta-glucosyltransferase activity, uridine diphosphoglucose-ketone cyanohydrin glucosyltransferase activity, uridine diphosphoglucose-ketone glucosyltransferase activity Relationships: is a type of UDP-glycosyltransferase activity [GO:0008194]; is_a hexosyltransferase activity [GO:0016758] Definition: Catalysis of the reaction: UDP-glucose + 2-hydroxy-2-methylpropanenitrile = UDP + linamarin.